{
  "gene_symbol": "CRIPTO3",
  "gene": "UniProtKB:P51864",
  "term_label": "blood vessel development",
  "term_id": "GO:0001568",
  "gene_name": "Putative teratocarcinoma-derived growth factor 3"
}